{
  "term_id": "GO:0045861",
  "gene_name": "Serine protease inhibitor Kazal-type 6",
  "term_label": "negative regulation of proteolysis",
  "gene": "UniProtKB:Q6UWN8",
  "gene_symbol": "SPINK6"
}